{
  "gene_symbol": "UGT1A9",
  "term_id": "GO:0008194",
  "term_label": "UDP-glycosyltransferase activity",
  "gene": "UniProtKB:O60656",
  "gene_name": "UDP-glucuronosyltransferase 1A9"
}